{
  "gene_name": "Interferon alpha-10",
  "term_id": "GO:0005615",
  "term_label": "extracellular space",
  "gene": "UniProtKB:P01566",
  "gene_symbol": "IFNA10"
}